{
  "term_id": "UNKNOWN:0001",
  "gene_symbol": "GVQW3",
  "term_label": "Unknown molecular function",
  "gene": "UniProtKB:Q3ZCU0",
  "gene_name": "Protein GVQW3"
}